{
  "term_id": "GO:0000978",
  "gene_symbol": "ZNF215",
  "gene": "UniProtKB:Q9UL58",
  "term_label": "RNA polymerase II cis-regulatory region sequence-specific DNA binding",
  "gene_name": "Zinc finger protein 215"
}